parental behavior [GO:0060746] (biological process) Subtypes: maternal behavior [GO:0042711], paternal behavior [GO:0042712], oral incubation [GO:0060747] Relationships: is a type of GO:0019098 Definition: A reproductive behavior in which a parent cares for and rears offspring. Sources: GOC:dph